{
  "term_label": "nucleus",
  "gene_name": "Transducin-like enhancer protein 7",
  "gene_symbol": "TLE7",
  "gene": "UniProtKB:A0A1W2PR48",
  "term_id": "GO:0005634"
}